{
  "gene_symbol": "MEAF6",
  "gene_name": "Chromatin modification-related protein MEAF6",
  "term_id": "UNKNOWN:0001",
  "term_label": "Unknown molecular function",
  "gene": "UniProtKB:Q9HAF1"
}